{
  "gene_name": "2-5A-dependent ribonuclease",
  "term_label": "defense response to virus",
  "gene_symbol": "RNASEL",
  "term_id": "GO:0051607",
  "gene": "UniProtKB:Q05823"
}